regulation of neuron apoptotic process [GO:0043523] (biological process) Subtypes: negative regulation of neuron apoptotic process [GO:0043524], GO:0043525, regulation of hippocampal neuron apoptotic process [GO:0110089], GO:1903376, regulation of endoplasmic reticulum stress-induced neuron intrinsic apoptotic signaling pathway [GO:1903381], regulation of outer hair cell apoptotic process [GO:1905585], regulation of motor neuron apoptotic process [GO:2000671] Sources: GOC:go_curators, GOC:mtg_apoptosis Definition: Any process that modulates the occurrence or rate of cell death by apoptotic process in neurons. Also known as: regulation of apoptosis of neuronal cells, regulation of apoptosis of neurons, regulation of neuron programmed cell death, regulation of neuronal cell programmed cell death, regulation of programmed cell death of neuronal cells, regulation of programmed cell death, neurons, regulation of neuron apoptosis Relationships: is a type of regulation of apoptotic process [GO:0042981]; regulates GO:0051402